{
  "gene": "UniProtKB:P62877",
  "term_label": "protein ubiquitination",
  "gene_symbol": "RBX1",
  "term_id": "GO:0016567",
  "gene_name": "E3 ubiquitin-protein ligase RBX1"
}